{
  "gene": "UniProtKB:Q8IZC6",
  "gene_symbol": "COL27A1",
  "term_id": "GO:0030020",
  "gene_name": "Collagen alpha-1(XXVII) chain",
  "term_label": "extracellular matrix structural constituent conferring tensile strength"
}